{
  "gene": "UniProtKB:Q6ZW05",
  "term_label": "Unknown molecular function",
  "gene_symbol": "PTCHD4",
  "term_id": "UNKNOWN:0001",
  "gene_name": "Patched domain-containing protein 4"
}